{
  "gene_symbol": "CRYBA1",
  "gene": "UniProtKB:P05813",
  "gene_name": "Beta-crystallin A3",
  "term_id": "GO:0005212",
  "term_label": "structural constituent of eye lens"
}